{
  "gene": "UniProtKB:Q14498",
  "term_label": "Unknown cellular component",
  "gene_name": "RNA-binding protein 39",
  "gene_symbol": "RBM39",
  "term_id": "UNKNOWN:0003"
}